RITS complex [GO:0030958] (cellular component) Definition: A protein complex required for heterochromatin assembly; contains an Argonaute homolog, a chromodomain protein, and at least one additional protein; named for RNA-induced initiation of transcriptional gene silencing. References: PMID:14704433 Relationships: is a type of RNAi effector complex [GO:0031332]; is a type of nuclear protein-containing complex [GO:0140513]; BFO_0000050 GO:0000228; is part of heterochromatin [GO:0000792]